{
  "gene_name": "Calcineurin B homologous protein 3",
  "gene": "UniProtKB:Q96BS2",
  "gene_symbol": "TESC",
  "term_id": "GO:0072659",
  "term_label": "protein localization to plasma membrane"
}